{
  "gene_name": "Dedicator of cytokinesis protein 7",
  "term_label": "regulation of Rho protein signal transduction",
  "term_id": "GO:0035023",
  "gene_symbol": "DOCK7",
  "gene": "UniProtKB:Q96N67"
}